{
  "gene_name": "Coiled-coil and C2 domain-containing protein 2A",
  "term_id": "GO:0035869",
  "term_label": "ciliary transition zone",
  "gene_symbol": "CC2D2A",
  "gene": "UniProtKB:Q9P2K1"
}